{
  "term_id": "GO:0003400",
  "term_label": "regulation of COPII vesicle coating",
  "gene_symbol": "SAR1A",
  "gene_name": "GTP-binding protein SAR1a",
  "gene": "UniProtKB:Q9NR31"
}